{
  "gene_name": "Protein GPR108",
  "gene_symbol": "GPR108",
  "term_id": "UNKNOWN:0001",
  "term_label": "Unknown molecular function",
  "gene": "UniProtKB:Q9NPR9"
}